{
  "term_id": "UNKNOWN:0002",
  "gene": "UniProtKB:A6NI28",
  "gene_symbol": "ARHGAP42",
  "gene_name": "Rho GTPase-activating protein 42",
  "term_label": "Unknown biological process"
}